{
  "gene_symbol": "OR4N5",
  "gene": "UniProtKB:Q8IXE1",
  "term_id": "GO:0004984",
  "term_label": "olfactory receptor activity",
  "gene_name": "Olfactory receptor 4N5"
}